{
  "gene_name": "Succinate receptor 1",
  "gene": "UniProtKB:Q9BXA5",
  "term_label": "signaling receptor activity",
  "term_id": "GO:0038023",
  "gene_symbol": "SUCNR1"
}